{
  "gene_symbol": "PTPN18",
  "term_id": "UNKNOWN:0002",
  "gene": "UniProtKB:Q99952",
  "term_label": "Unknown biological process",
  "gene_name": "Tyrosine-protein phosphatase non-receptor type 18"
}